{
  "gene": "UniProtKB:P30559",
  "term_label": "vasopressin receptor activity",
  "gene_name": "Oxytocin receptor",
  "term_id": "GO:0005000",
  "gene_symbol": "OXTR"
}